{
  "gene": "UniProtKB:Q9BX66",
  "gene_name": "Sorbin and SH3 domain-containing protein 1",
  "term_id": "GO:0005886",
  "gene_symbol": "SORBS1",
  "term_label": "plasma membrane"
}